{
  "term_id": "UNKNOWN:0001",
  "gene_name": "Uncharacterized protein C1orf141",
  "gene_symbol": "C1orf141",
  "term_label": "Unknown molecular function",
  "gene": "UniProtKB:Q5JVX7"
}